{
  "gene_name": "Immunoglobulin superfamily DCC subclass member 4",
  "term_label": "cell-cell adhesion",
  "gene_symbol": "IGDCC4",
  "gene": "UniProtKB:Q8TDY8",
  "term_id": "GO:0098609"
}